{
  "gene_symbol": "SLC24A1",
  "gene": "UniProtKB:O60721",
  "gene_name": "Sodium_potassium_calcium exchanger 1",
  "term_label": "calcium, potassium:sodium antiporter activity",
  "term_id": "GO:0008273"
}